{
  "term_label": "RNA polymerase II cis-regulatory region sequence-specific DNA binding",
  "gene_name": "Zinc finger protein 724",
  "gene": "UniProtKB:A8MTY0",
  "term_id": "GO:0000978",
  "gene_symbol": "ZNF724"
}